{
  "gene_symbol": "C9orf57",
  "gene": "UniProtKB:Q5W0N0",
  "term_label": "Unknown biological process",
  "term_id": "UNKNOWN:0002",
  "gene_name": "Uncharacterized protein C9orf57"
}